N-acetylgalactosamine-4-sulfatase activity [GO:0003943] (molecular function) Definition: Catalysis of the hydrolysis of the 4-sulfate groups of the N-acetyl-D-galactosamine 4-sulfate units of chondroitin sulfate and dermatan sulfate. Relationships: is a type of sulfuric ester hydrolase activity [GO:0008484] Also known as: chondroitinsulfatase, N-acetylgalactosamine-4-sulphatase activity, arylsulfatase B, N-acetyl-D-galactosamine-4-sulfate 4-sulfohydrolase activity, N-acetylgalactosamine 4-sulfate sulfohydrolase activity, acetylgalactosamine 4-sulfatase activity Sources: EC:3.1.6.12